{
  "gene_symbol": "TRAV5",
  "term_id": "GO:0009617",
  "term_label": "response to bacterium",
  "gene_name": "T cell receptor alpha variable 5",
  "gene": "UniProtKB:A0A0B4J249"
}